gibberellic acid mediated signaling pathway, G-alpha-independent [GO:0042390] (biological process) Relationships: is a type of GO:0009740 Definition: The series of molecular signals mediated by the detection of gibberellic acid and not dependent on the coupling of the alpha subunit of G proteins to the hormone receptors. References: PMID:11027362 Sources: GOC:pj Also known as: gibberellic acid mediated signalling, G-alpha-independent